{
  "term_id": "UNKNOWN:0003",
  "gene_symbol": "LRRC66",
  "gene_name": "Leucine-rich repeat-containing protein 66",
  "gene": "UniProtKB:Q68CR7",
  "term_label": "Unknown cellular component"
}